regulation of photoreceptor cell axon guidance [GO:2000289] (biological process) Also known as: regulation of photoreceptor cell axon pathfinding Sources: GOC:mah Definition: Any process that modulates the frequency, rate or extent of photoreceptor cell axon guidance. Relationships: is a type of regulation of axon guidance [GO:1902667]; regulates photoreceptor cell axon guidance [GO:0072499]